negative regulation of tumor necrosis factor (ligand) superfamily member 11 production [GO:2000308] (biological process) Relationships: is a type of GO:1903556; is_a regulation of tumor necrosis factor (ligand) superfamily member 11 production [GO:2000307]; negatively regulates tumor necrosis factor (ligand) superfamily member 11 production [GO:0072535] Sources: GOC:BHF, GOC:mah Also known as: negative regulation of RANKL production, negative regulation of TNFSF11 production Definition: Any process that stops, prevents or reduces the frequency, rate or extent of tumor necrosis factor (ligand) superfamily member 11 production.